sympathetic neuron axon guidance [GO:0097492] (BP) Relationships: is a type of GO:0007411 Definition: The chemotaxis process that directs the migration of a sympathetic neuron axon growth cone to a specific target site in response to a combination of attractive and repulsive cues. References: PMID:22790009 Sources: GOC:BHF, GOC:rl Also known as: sympathetic neuron axon pathfinding, sympathetic neuron axon growth cone guidance, sympathetic neuron axon chemotaxis